{
  "gene_symbol": "A0A096LPG2",
  "gene": "UniProtKB:A0A096LPG2",
  "term_label": "Unknown biological process",
  "gene_name": "Uncharacterized protein",
  "term_id": "UNKNOWN:0002"
}